{
  "gene": "UniProtKB:Q9UJ98",
  "term_label": "meiotic cohesin complex",
  "gene_name": "Cohesin subunit SA-3",
  "term_id": "GO:0030893",
  "gene_symbol": "STAG3"
}